{
  "gene_name": "Sodium-dependent noradrenaline transporter",
  "term_id": "GO:0030424",
  "gene_symbol": "SLC6A2",
  "gene": "UniProtKB:P23975",
  "term_label": "axon"
}